extracellular matrix disassembly [GO:0022617] (biological process) Regulation: regulated by regulation of extracellular matrix disassembly [GO:0010715]; negatively regulated by negative regulation of extracellular matrix disassembly [GO:0010716]; RO_0002213 by positive regulation of extracellular matrix disassembly [GO:0090091] Relationships: is a type of GO:0022411; is_a extracellular matrix organization [GO:0030198] Sources: GOC:jid Subtypes: basement membrane disassembly [GO:0034769], GO:0098786 Definition: A process that results in the breakdown of the extracellular matrix.